positive regulation of Fas signaling pathway [GO:1902046] (biological process) Also known as: positive regulation of Apo-1 signaling pathway, positive regulation of CD95 signaling pathway, positive regulation of Fas receptor signaling pathway, positive regulation of FasR signaling pathway, up regulation of Apo-1 signaling pathway, up regulation of CD95 signaling pathway, up regulation of Fas receptor signaling pathway, up regulation of Fas signaling pathway, up regulation of FasR signaling pathway, up-regulation of Apo-1 signaling pathway, up-regulation of CD95 signaling pathway, up-regulation of Fas receptor signaling pathway, up-regulation of Fas signaling pathway, up-regulation of FasR signaling pathway, upregulation of Apo-1 signaling pathway, upregulation of CD95 signaling pathway, upregulation of Fas receptor signaling pathway, upregulation of Fas signaling pathway, upregulation of FasR signaling pathway, activation of Apo-1 signaling pathway, activation of CD95 signaling pathway, activation of FAS ligand-Fas signaling pathway, activation of Fas receptor signaling pathway, activation of Fas signaling pathway, activation of Fas-FasL signaling pathway, activation of FasR signaling pathway, positive regulation of FAS ligand-Fas signaling pathway, positive regulation of Fas-FasL signaling pathway, up regulation of FAS ligand-Fas signaling pathway, up regulation of Fas-FasL signaling pathway, up-regulation of FAS ligand-Fas signaling pathway, up-regulation of Fas-FasL signaling pathway, upregulation of FAS ligand-Fas signaling pathway, upregulation of Fas-FasL signaling pathway, activation of FasL signaling pathway, positive regulation of FasL signaling pathway, up regulation of FasL signaling pathway, up-regulation of FasL signaling pathway, upregulation of FasL signaling pathway References: PMID:17245429 Sources: GOC:TermGenie Relationships: is a type of positive regulation of signal transduction [GO:0009967]; is a type of regulation of Fas signaling pathway [GO:1902044]; RO_0002213 GO:0036337 Definition: Any process that activates or increases the frequency, rate or extent of Fas signaling pathway.